stomium development [GO:0080166] (biological process) Sources: GOC:tb Definition: The process whose specific outcome is the progression of the stomium over time, from its formation to the mature structure. A stomium is a fissure or pore in the anther lobe through which the pollen is released. Relationships: is a type of developmental process involved in reproduction [GO:0003006]; is a type of cellular process involved in reproduction in multicellular organism [GO:0022412]; is a type of GO:0048856; is part of anther development [GO:0048653]